{
  "gene": "UniProtKB:P25089",
  "term_id": "GO:0006954",
  "gene_name": "N-formyl peptide receptor 3",
  "gene_symbol": "FPR3",
  "term_label": "inflammatory response"
}